negative regulation of age-related resistance [GO:1904249] (biological process) Definition: Any process that stops, prevents or reduces the extent of age-related resistance. References: PMID:19694953 Sources: GOC:TermGenie, GO_REF:0000058 Relationships: is_a negative regulation of innate immune response [GO:0045824]; is a type of negative regulation of developmental process [GO:0051093]; is a type of GO:1904248; negatively regulates age-related resistance [GO:0090644] Also known as: down regulation of ARR, down regulation of age-related resistance, down-regulation of ARR, down-regulation of age-related resistance, downregulation of ARR, downregulation of age-related resistance, negative regulation of ARR, down regulation of adult seedling resistance, down regulation of flowering-induced resistance, down regulation of mature seedling resistance, down regulation of senescence-induced resistance, down-regulation of adult seedling resistance, down-regulation of flowering-induced resistance, down-regulation of mature seedling resistance, down-regulation of senescence-induced resistance, downregulation of adult seedling resistance, downregulation of flowering-induced resistance, downregulation of mature seedling resistance, downregulation of senescence-induced resistance, inhibition of ARR, inhibition of adult seedling resistance, inhibition of age-related resistance, inhibition of flowering-induced resistance, inhibition of mature seedling resistance, inhibition of senescence-induced resistance, negative regulation of adult seedling resistance, negative regulation of flowering-induced resistance, negative regulation of mature seedling resistance, negative regulation of senescence-induced resistance